{
  "gene_symbol": "HES1",
  "term_id": "GO:0000122",
  "gene": "UniProtKB:Q14469",
  "gene_name": "Transcription factor HES-1",
  "term_label": "negative regulation of transcription by RNA polymerase II"
}